{
  "gene_symbol": "ARMC9",
  "gene": "UniProtKB:Q7Z3E5",
  "term_label": "ciliary tip",
  "term_id": "GO:0097542",
  "gene_name": "LisH domain-containing protein ARMC9"
}